peroxisome localization [GO:0060151] (biological process) References: PMID:16449325 Sources: GOC:dph Relationships: is a type of GO:0051640 Definition: Any process in which a peroxisome is transported to, and/or maintained in, a specific location. A peroxisome is a small membrane-bounded organelle that uses dioxygen (O2) to oxidize organic molecules. Also known as: peroxisome localisation Subtypes: microtubule-based peroxisome localization [GO:0060152], endoplasmic reticulum-peroxisome tethering [GO:0062095]